L-lysine transport [GO:1902022] (biological process) Definition: The directed movement of a L-lysine into, out of or within a cell, or between cells, by means of some agent such as a transporter or pore. References: PMID:22822152 Sources: GOC:TermGenie, GOC:kmv Relationships: is a type of organic cation transport [GO:0015695]; is a type of GO:0015807 Subtypes: lysine transport [GO:0015819], L-lysine transmembrane transport [GO:1903401]